{
  "gene_symbol": "FAM9B",
  "term_label": "spermatid development",
  "gene": "UniProtKB:Q8IZU0",
  "gene_name": "Protein FAM9B",
  "term_id": "GO:0007286"
}